cell surface receptor protein tyrosine phosphatase signaling pathway [GO:0007185] (BP) Sources: GOC:mah, GOC:signaling Also known as: transmembrane receptor protein tyrosine phosphatase signaling pathway, transmembrane receptor protein tyrosine phosphatase signalling pathway Relationships: is a type of enzyme-linked receptor protein signaling pathway [GO:0007167] Definition: The series of molecular signals initiated by an extracellular ligand binding to a receptor on the surface of the target cell where the receptor possesses protein tyrosine phosphatase activity, and ending with the regulation of a downstream cellular process, e.g. transcription.